{
  "gene_symbol": "TEFM",
  "gene": "UniProtKB:Q96QE5",
  "gene_name": "Transcription elongation factor, mitochondrial",
  "term_label": "mitochondrial nucleoid",
  "term_id": "GO:0042645"
}